{
  "term_id": "GO:0006357",
  "gene": "UniProtKB:P31249",
  "gene_name": "Homeobox protein Hox-D3",
  "term_label": "regulation of transcription by RNA polymerase II",
  "gene_symbol": "HOXD3"
}